{
  "term_label": "endoplasmic reticulum to Golgi vesicle-mediated transport",
  "gene_symbol": "YKT6",
  "term_id": "GO:0006888",
  "gene": "UniProtKB:O15498",
  "gene_name": "Synaptobrevin homolog YKT6"
}